{
  "term_label": "establishment of protein localization to organelle",
  "gene": "UniProtKB:P11279",
  "term_id": "GO:0072594",
  "gene_symbol": "LAMP1",
  "gene_name": "Lysosome-associated membrane glycoprotein 1"
}